UTP thiamine diphosphokinase activity [GO:0141200] (molecular function) References: PMID:38547260 Sources: RHEA:79423 Relationships: is a type of diphosphotransferase activity [GO:0016778] Definition: Catalysis of the reaction: UTP + thiamine = UMP + thiamine diphosphate.